{
  "term_id": "GO:0030154",
  "gene_name": "Transcription factor Spi-C",
  "term_label": "cell differentiation",
  "gene": "UniProtKB:Q8N5J4",
  "gene_symbol": "SPIC"
}